{
  "gene_name": "GSK3B-interacting protein",
  "term_label": "protein kinase A binding",
  "gene": "UniProtKB:Q9P0R6",
  "term_id": "GO:0051018",
  "gene_symbol": "GSKIP"
}